ubiquinone-6 binding [GO:1900995] (molecular function) Relationships: is a type of ubiquinone binding [GO:0048039] Sources: GOC:TermGenie, GOC:al Definition: Binding to ubiquinone-6. Ubiquinone-6 is a ubiquinone compound having a (2E,6E,10E,14E,18E)-3,7,11,15,19,23-hexamethyltetracosa-2,6,10,14,18,22-hexaen-1-yl substituent at position 2.